regulation of acrosomal vesicle exocytosis [GO:2000367] (biological process) Definition: Any process that modulates the frequency, rate or extent of acrosomal vesicle exocytosis. Sources: GOC:obol Also known as: regulation of acrosome exocytosis, regulation of acrosomal granule exocytosis Relationships: is a type of regulation of calcium ion-dependent exocytosis [GO:0017158]; regulates acrosomal vesicle exocytosis [GO:0060478] Subtypes: GO:2000368